{
  "gene_symbol": "CCL1",
  "gene_name": "C-C motif chemokine 1",
  "gene": "UniProtKB:P22362",
  "term_label": "extracellular space",
  "term_id": "GO:0005615"
}